subpallium glioblast cell division [GO:0021850] (biological process) Definition: The division of glioblasts in the subpallium. These cells will give rise to oligodendrocytes. Also known as: glioblast cell division in subpallium, glioblast division in ventral telencephalon Relationships: is a type of glioblast division [GO:0048860]; is part of subpallium cell proliferation in forebrain [GO:0022012] References: PMID:12626695 Sources: GOC:cls, GOC:dgh, GOC:dph, GOC:jid, GO_REF:0000021